{
  "gene": "UniProtKB:Q9NXF8",
  "term_id": "GO:0072659",
  "gene_name": "Palmitoyltransferase ZDHHC7",
  "term_label": "protein localization to plasma membrane",
  "gene_symbol": "ZDHHC7"
}